{
  "term_label": "Unknown cellular component",
  "gene": "UniProtKB:Q3MJ62",
  "term_id": "UNKNOWN:0003",
  "gene_symbol": "ZSCAN23",
  "gene_name": "Zinc finger and SCAN domain-containing protein 23"
}